{
  "gene": "UniProtKB:Q495M3",
  "gene_symbol": "SLC36A2",
  "term_id": "GO:0005280",
  "gene_name": "Proton-coupled amino acid transporter 2",
  "term_label": "amino acid:proton symporter activity"
}